{
  "gene": "UniProtKB:Q15773",
  "term_label": "Unknown molecular function",
  "term_id": "UNKNOWN:0001",
  "gene_name": "Myeloid leukemia factor 2",
  "gene_symbol": "MLF2"
}